{
  "gene_name": "LysM and putative peptidoglycan-binding domain-containing protein 2",
  "gene": "UniProtKB:Q8IV50",
  "gene_symbol": "LYSMD2",
  "term_id": "UNKNOWN:0003",
  "term_label": "Unknown cellular component"
}